{
  "term_id": "GO:0044818",
  "gene_symbol": "CHFR",
  "gene_name": "E3 ubiquitin-protein ligase CHFR",
  "gene": "UniProtKB:Q96EP1",
  "term_label": "mitotic G2/M transition checkpoint"
}